{
  "term_id": "UNKNOWN:0003",
  "gene_name": "POLG alternative reading frame",
  "gene": "UniProtKB:A0A3B3IS91",
  "gene_symbol": "POLGARF",
  "term_label": "Unknown cellular component"
}